zinc ion sequestering activity [GO:0140486] (molecular function) Definition: Binding to a zinc ion to prevent it from interacting with other partners or to inhibit its localization to the area of the cell or complex where it is active. References: PMID:12050156 Relationships: is a type of metal ion sequestering activity [GO:0140487]; has part GO:0008270